trans-synaptic signaling [GO:0099537] (biological process) Subtypes: GO:0098916, GO:0098917, GO:0099157, trans-synaptic signaling by BDNF [GO:0099191], trans-synaptic signaling by neuropeptide [GO:0099540], GO:0099541, GO:0099543, trans-synaptic signaling by trans-synaptic complex [GO:0099545], trans-synaptic signaling, modulating synaptic transmission [GO:0099550] Regulation: regulated by regulation of trans-synaptic signaling [GO:0099177] Sources: GOC:dos Definition: Cell-cell signaling in either direction across the synaptic cleft. Relationships: is a type of synaptic signaling [GO:0099536]